selenocysteine metabolic process [GO:0016259] (biological process) Also known as: selenocysteine metabolism Sources: GOC:go_curators, ISBN:0198506732 Definition: The chemical reactions and pathways involving selenocysteine, an essential component of glutathione peroxidase and some other proteins. Subtypes: selenocysteine biosynthetic process [GO:0016260], selenocysteine catabolic process [GO:0016261] Relationships: is a type of alpha-amino acid metabolic process [GO:1901605]